symbiont-mediated response to host defenses [GO:0052200] (biological process) Relationships: is a type of GO:0075136 Note: Note that this term is used to annotate gene products of the symbiont. Sources: GOC:mtg_pamgo_17jul06 Definition: Any process that results in a change in state or activity of a cell or an organism (in terms of movement, secretion, enzyme production, gene expression, etc.) as a result of detecting the defenses of the host organism. The host is defined as the larger of the organisms involved in a symbiotic interaction. Also known as: response to host defenses, maintenance of symbiont tolerance to host defense molecules, response of symbiont to host defense molecules, response to host defense molecules Subtypes: GO:0030682, response to host immune response [GO:0052572], effector-mediated perturbation of host defenses by symbiont [GO:0140415]